{
  "term_id": "UNKNOWN:0002",
  "gene_name": "Lipocalin-like 1 protein",
  "gene_symbol": "LCNL1",
  "term_label": "Unknown biological process",
  "gene": "UniProtKB:Q6ZST4"
}